{
  "term_id": "GO:0006589",
  "gene_name": "Dopamine beta-hydroxylase",
  "term_label": "octopamine biosynthetic process",
  "gene_symbol": "DBH",
  "gene": "UniProtKB:P09172"
}